{
  "term_label": "Unknown molecular function",
  "gene_name": "Small integral membrane protein 10",
  "gene": "UniProtKB:Q96HG1",
  "term_id": "UNKNOWN:0001",
  "gene_symbol": "SMIM10"
}